{
  "gene": "UniProtKB:Q8WVV5",
  "term_label": "T cell receptor signaling pathway",
  "term_id": "GO:0050852",
  "gene_symbol": "BTN2A2",
  "gene_name": "Butyrophilin subfamily 2 member A2"
}